{
  "term_label": "Unknown molecular function",
  "gene": "UniProtKB:P55082",
  "term_id": "UNKNOWN:0001",
  "gene_name": "Microfibril-associated glycoprotein 3",
  "gene_symbol": "MFAP3"
}